alpha6-beta4 integrin-laminin 5 complex [GO:0070334] (cellular component) Definition: A protein complex that consists of an alpha6-beta4 integrin complex bound to laminin 5. References: PMID:7556090 Sources: GOC:mah Also known as: alpha6-beta4 integrin-laminin-332 complex, ITGA6-ITGB4-LAMA5 complex Relationships: is a type of plasma membrane protein complex [GO:0098797]